{
  "term_id": "GO:0005737",
  "gene": "UniProtKB:Q96MN2",
  "gene_name": "NACHT, LRR and PYD domains-containing protein 4",
  "term_label": "cytoplasm",
  "gene_symbol": "NLRP4"
}